{
  "gene_name": "A-kinase anchor protein 1, mitochondrial",
  "gene_symbol": "AKAP1",
  "term_id": "GO:0034237",
  "term_label": "protein kinase A regulatory subunit binding",
  "gene": "UniProtKB:Q92667"
}